enucleate erythrocyte development [GO:0048822] (biological process) Also known as: enucleate RBC development, enucleate red blood cell development Definition: The process aimed at the progression of an enucleate erythrocyte over time, from initial commitment of the cell to a specific fate, to the fully functional differentiated cell. Sources: GOC:devbiol Relationships: is a type of erythrocyte development [GO:0048821]; is part of enucleate erythrocyte differentiation [GO:0043353]